{
  "term_label": "phosphate ion transmembrane transport",
  "term_id": "GO:0035435",
  "gene_name": "Glucose-6-phosphate exchanger SLC37A1",
  "gene_symbol": "SLC37A1",
  "gene": "UniProtKB:P57057"
}